{
  "gene": "UniProtKB:P56199",
  "term_label": "cell surface",
  "gene_name": "Integrin alpha-1",
  "gene_symbol": "ITGA1",
  "term_id": "GO:0009986"
}